{
  "gene_symbol": "SHISA4",
  "term_label": "Unknown cellular component",
  "gene_name": "Protein shisa-4",
  "gene": "UniProtKB:Q96DD7",
  "term_id": "UNKNOWN:0003"
}